{
  "term_id": "GO:0007338",
  "gene_symbol": "PRND",
  "gene": "UniProtKB:Q9UKY0",
  "term_label": "single fertilization",
  "gene_name": "Prion-like protein doppel"
}